{
  "term_label": "3',5'-cyclic-AMP phosphodiesterase activity",
  "gene_name": "cAMP and cAMP-inhibited cGMP 3',5'-cyclic phosphodiesterase 10A",
  "gene": "UniProtKB:Q9Y233",
  "term_id": "GO:0004115",
  "gene_symbol": "PDE10A"
}